bacterial-type RNA polymerase holo enzyme binding [GO:0001108] (molecular function) Relationships: is a type of basal transcription machinery binding [GO:0001098] Sources: GOC:txnOH Also known as: basal bacterial-type RNA polymerase transcription machinery binding Definition: Binding to a component of the basal transcription machinery which is composed of a bacterial-type RNA polymerase core enzyme and a sigma factor, the minimal set of factors required for formation of the preinitiation complex (PIC) by a bacterial-type RNA polymerase.